{
  "term_label": "nucleus",
  "gene_name": "5'-AMP-activated protein kinase subunit gamma-3",
  "gene_symbol": "PRKAG3",
  "gene": "UniProtKB:Q9UGI9",
  "term_id": "GO:0005634"
}